myoblast proliferation involved in skeletal muscle regeneration [GO:0014844] (biological process) Definition: The multiplication or reproduction of myoblasts, resulting in the expansion of the cell population. This occurs as part of skeletal muscle regeneration. A myoblast is a mononucleate cell type that, by fusion with other myoblasts, gives rise to the myotubes that eventually develop into skeletal muscle fibers. References: PMID:16607119 Sources: CL:0000056, GOC:ef, GOC:mtg_muscle Relationships: is a type of myoblast proliferation [GO:0051450]; is part of skeletal muscle tissue regeneration [GO:0043403]